{
  "term_id": "UNKNOWN:0001",
  "gene_name": "Cilia- and flagella-associated protein HOATZ",
  "gene_symbol": "HOATZ",
  "term_label": "Unknown molecular function",
  "gene": "UniProtKB:Q6PI97"
}